{
  "term_id": "GO:0000281",
  "term_label": "mitotic cytokinesis",
  "gene": "UniProtKB:O75116",
  "gene_name": "Rho-associated protein kinase 2",
  "gene_symbol": "ROCK2"
}